{
  "gene_name": "Programmed cell death 1 ligand 2",
  "gene": "UniProtKB:Q9BQ51",
  "gene_symbol": "PDCD1LG2",
  "term_label": "positive regulation of T cell proliferation",
  "term_id": "GO:0042102"
}